{
  "gene": "UniProtKB:O00222",
  "term_label": "G protein-coupled glutamate receptor signaling pathway",
  "gene_symbol": "GRM8",
  "gene_name": "Metabotropic glutamate receptor 8",
  "term_id": "GO:0007216"
}